{
  "term_label": "voltage-gated calcium channel complex",
  "gene_name": "Voltage-dependent L-type calcium channel subunit alpha-1D",
  "gene_symbol": "CACNA1D",
  "term_id": "GO:0005891",
  "gene": "UniProtKB:Q01668"
}